{
  "gene_name": "HCLS1-binding protein 3",
  "gene": "UniProtKB:Q53T59",
  "term_id": "UNKNOWN:0001",
  "term_label": "Unknown molecular function",
  "gene_symbol": "HS1BP3"
}